{
  "term_label": "RNA polymerase II transcription regulatory region sequence-specific DNA binding",
  "gene_symbol": "CREBRF",
  "term_id": "GO:0000977",
  "gene": "UniProtKB:Q8IUR6",
  "gene_name": "CREB3 regulatory factor"
}